atrial cardiac muscle cell fate commitment [GO:0060924] (biological process) Sources: GOC:mtg_heart Definition: The commitment of cells to atrial cardiac muscle cell fates and their capacity to differentiate into cardiac muscle cells of the atrium. Cardiac muscle cells are striated muscle cells that are responsible for heart contraction. Also known as: atrial heart muscle cell fate commitment, atrial cardiomyocyte cell fate commitment Relationships: is a type of GO:0060923; is part of GO:0055011